{
  "gene": "UniProtKB:Q7Z3U7",
  "term_label": "protein targeting to vacuole",
  "gene_symbol": "MON2",
  "gene_name": "Protein MON2 homolog",
  "term_id": "GO:0006623"
}